{
  "gene_symbol": "ANXA10",
  "term_id": "GO:0012506",
  "gene": "UniProtKB:Q9UJ72",
  "gene_name": "Annexin A10",
  "term_label": "vesicle membrane"
}